{
  "gene_symbol": "SOX5",
  "gene": "UniProtKB:P35711",
  "gene_name": "Transcription factor SOX-5",
  "term_id": "GO:0005634",
  "term_label": "nucleus"
}